{
  "gene_name": "Calcineurin B homologous protein 1",
  "gene_symbol": "CHP1",
  "term_label": "membrane docking",
  "term_id": "GO:0022406",
  "gene": "UniProtKB:Q99653"
}